small molecule binding [GO:0036094] (molecular function) Note: Small molecules in GO include monosaccharides but exclude disaccharides and polysaccharides. Sources: GOC:curators, GOC:pde, GOC:pm Subtypes: GO:0000035, selenium binding [GO:0008430], oxygen binding [GO:0019825], vitamin binding [GO:0019842], urea binding [GO:0033219], 2-aminoethylphosphonate binding [GO:0033226], ion binding [GO:0043167], organic acid binding [GO:0043177], alcohol binding [GO:0043178], poly(3-hydroxyalkanoate) binding [GO:0043287], hydroxyapatite binding [GO:0046848], monosaccharide binding [GO:0048029], quinone binding [GO:0048038], ice binding [GO:0050825], quaternary ammonium group binding [GO:0050997], GO:0051540, carbon monoxide binding [GO:0070025], GO:0070026, alkene binding [GO:0072328], GO:1901363, GO:1902670, tetrahydrofolyl-poly(glutamate) polymer binding [GO:1904493] Relationships: is a type of binding [GO:0005488] Definition: Binding to a small molecule, any low molecular weight, monomeric, non-encoded molecule.